{
  "gene_symbol": "ABCD4",
  "term_label": "long-chain fatty acid transmembrane transporter activity",
  "term_id": "GO:0005324",
  "gene_name": "Lysosomal cobalamin transporter ABCD4",
  "gene": "UniProtKB:O14678"
}